{
  "term_id": "GO:0007219",
  "gene_name": "Disintegrin and metalloproteinase domain-containing protein 17",
  "gene": "UniProtKB:P78536",
  "gene_symbol": "ADAM17",
  "term_label": "Notch signaling pathway"
}